mitotic G2 phase [GO:0000085] (biological process) Definition: The cell cycle 'gap' phase which is the interval between the completion of DNA synthesis and the beginning of DNA segregation by mitosis. Note: Note that this term should not be used for direct annotation. If you are trying to make an annotation to x phase, it is likely that the correct annotation is 'regulation of x/y phase transition' or to a process which occurs during the reported phase (i.e mitotic DNA replication for mitotic S-phase). To capture the phase when a specific location or process is observed, the phase term can be used in an annotation extension (PMID:24885854) applied to a cellular component term (with the relation exists_during) or a biological process term (with the relation happens_during). Sources: GOC:mtg_cell_cycle Also known as: G2 phase of mitotic cell cycle Relationships: is a type of G2 phase [GO:0051319]; is part of mitotic interphase [GO:0051329]